establishment of endoplasmic reticulum localization to postsynapse [GO:0099089] (biological process) Also known as: establishment of ER localization to postsynapse Relationships: is a type of establishment of ER localization [GO:0051686] References: PMID:21151132 Sources: GOC:dos Definition: The directed movement of endoplasmic reticulum into a postsynaptic compartment such as a dendritic spine.